{
  "term_id": "GO:0032869",
  "gene_symbol": "LPIN2",
  "gene_name": "Phosphatidate phosphatase LPIN2",
  "term_label": "cellular response to insulin stimulus",
  "gene": "UniProtKB:Q92539"
}